tRNA wobble base lysidine biosynthesis [GO:0002136] (BP) References: PMID:15894617 Definition: The process in which the carbonyl of cytosine at position 34 of a tRNA is post-transcriptionally replaced by lysine. Relationships: is a type of GO:0002101 Note: Exclusively located at the anticodon wobble position (i.e., position 34) of eubacterial and some organellar tRNAIle2. This modification converts the codon specificity from AUG to AUA, and it also converts the aminoacylation specificity of the tRNA from methionine to isoleucine. Requires ATP.